regulation of neural retina development [GO:0061074] (biological process) Relationships: is a type of regulation of developmental process [GO:0050793]; regulates neural retina development [GO:0003407] Definition: Any process that modulates the rate, frequency, or extent of neural retina development, the progression of the neural retina over time from its initial formation to the mature structure. The neural retina is the part of the retina that contains neurons and photoreceptor cells. Subtypes: positive regulation of neural retina development [GO:0061075], negative regulation of neural retina development [GO:0061076] Sources: GOC:dph